{
  "gene_symbol": "NR1D1",
  "term_id": "GO:0000978",
  "gene": "UniProtKB:P20393",
  "term_label": "RNA polymerase II cis-regulatory region sequence-specific DNA binding",
  "gene_name": "Nuclear receptor subfamily 1 group D member 1"
}